{
  "gene": "UniProtKB:Q8NAP1",
  "gene_symbol": "CASTOR3P",
  "gene_name": "Putative protein CASTOR3P",
  "term_id": "GO:1903577",
  "term_label": "cellular response to L-arginine"
}